{
  "gene_name": "Platelet-derived growth factor subunit B",
  "term_id": "GO:0030335",
  "gene": "UniProtKB:P01127",
  "gene_symbol": "PDGFB",
  "term_label": "positive regulation of cell migration"
}